proximal tubule development [GO:0072014] (biological process) Relationships: is_a nephron tubule development [GO:0072080] Subtypes: GO:0035776, mesonephric proximal tubule development [GO:0061275], metanephric proximal tubule development [GO:0072237] Definition: The process whose specific outcome is the progression of the proximal tubule over time, from its formation to the mature structure. In mammals, the proximal tubule is a nephron tubule that connects Bowman's capsule to the descending thin limb of the loop of Henle. It has a brush border epithelial morphology. Sources: GOC:mtg_kidney_jan10